{
  "term_id": "UNKNOWN:0003",
  "gene": "UniProtKB:Q8WW01",
  "gene_name": "tRNA-splicing endonuclease subunit Sen15",
  "term_label": "Unknown cellular component",
  "gene_symbol": "TSEN15"
}